{
  "term_id": "GO:0000981",
  "gene": "UniProtKB:Q8N8Y5",
  "gene_name": "Zinc finger protein 41 homolog",
  "gene_symbol": "ZFP41",
  "term_label": "DNA-binding transcription factor activity, RNA polymerase II-specific"
}